{
  "gene": "UniProtKB:Q92681",
  "term_label": "Unknown biological process",
  "term_id": "UNKNOWN:0002",
  "gene_symbol": "RSC1A1",
  "gene_name": "Regulatory solute carrier protein family 1 member 1"
}